3'-5' exonuclease activity [GO:0008408] (molecular function) Relationships: is a type of exonuclease activity [GO:0004527] Definition: Catalysis of the hydrolysis of ester linkages within nucleic acids by removing nucleotide residues from the 3' end. Subtypes: 3'-5'-RNA exonuclease activity [GO:0000175], 3'-5'-DNA exonuclease activity [GO:0008296] Sources: GOC:ai Also known as: 3'-5'-exonuclease activity